regulation of fibroblast growth factor production [GO:0090270] (BP) Definition: Any process that modulates the rate, frequency or extent of the appearance of a fibroblast growth factor due to biosynthesis or secretion following a cellular stimulus, resulting in an increase in its intracellular or extracellular levels. Subtypes: GO:0090271, negative regulation of fibroblast growth factor production [GO:0090272] Sources: GOC:BHF Relationships: is a type of regulation of cytokine production [GO:0001817]; regulates fibroblast growth factor production [GO:0090269]